{
  "gene_symbol": "NR1H4",
  "term_id": "GO:0005634",
  "gene": "UniProtKB:Q96RI1",
  "term_label": "nucleus",
  "gene_name": "Bile acid receptor"
}